{
  "term_label": "mitochondrion",
  "gene": "UniProtKB:Q96A26",
  "term_id": "GO:0005739",
  "gene_name": "Protein FAM162A",
  "gene_symbol": "FAM162A"
}